{
  "gene_name": "Potassium_sodium hyperpolarization-activated cyclic nucleotide-gated channel 2",
  "gene": "UniProtKB:Q9UL51",
  "term_id": "GO:0030424",
  "term_label": "axon",
  "gene_symbol": "HCN2"
}